{
  "term_id": "GO:0000981",
  "gene_symbol": "FOXJ3",
  "gene": "UniProtKB:Q9UPW0",
  "gene_name": "Forkhead box protein J3",
  "term_label": "DNA-binding transcription factor activity, RNA polymerase II-specific"
}